{
  "term_label": "DNA-binding transcription factor activity, RNA polymerase II-specific",
  "gene_name": "Transcription factor MafG",
  "gene": "UniProtKB:O15525",
  "term_id": "GO:0000981",
  "gene_symbol": "MAFG"
}